{
  "term_label": "Unknown biological process",
  "term_id": "UNKNOWN:0002",
  "gene_symbol": "OTUD6B",
  "gene": "UniProtKB:Q8N6M0",
  "gene_name": "Deubiquitinase OTUD6B"
}